positive regulation of oxidative stress-induced neuron intrinsic apoptotic signaling pathway [GO:1903378] (biological process) Definition: Any process that activates or increases the frequency, rate or extent of oxidative stress-induced neuron intrinsic apoptotic signaling pathway. Sources: GOC:PARL, GOC:TermGenie, GOC:bf, GO_REF:0000058 Also known as: positive regulation of neuron intrinsic apoptotic signaling pathway in response to oxidative stress, up regulation of neuron intrinsic apoptotic signaling pathway in response to oxidative stress, up-regulation of neuron intrinsic apoptotic signaling pathway in response to oxidative stress, upregulation of neuron intrinsic apoptotic signaling pathway in response to oxidative stress, activation of neuron intrinsic apoptotic signaling pathway in response to oxidative stress, activation of neuron apoptosis in response to oxidative stress, positive regulation of neuron apoptosis in response to oxidative stress, up regulation of neuron apoptosis in response to oxidative stress, up-regulation of neuron apoptosis in response to oxidative stress, upregulation of neuron apoptosis in response to oxidative stress Relationships: is a type of positive regulation of neuron apoptotic process [GO:0043525]; is a type of positive regulation of oxidative stress-induced intrinsic apoptotic signaling pathway [GO:1902177]; is a type of regulation of oxidative stress-induced neuron intrinsic apoptotic signaling pathway [GO:1903376]; positively regulates GO:0036480